{
  "gene_name": "X-linked retinitis pigmentosa GTPase regulator",
  "gene_symbol": "RPGR",
  "term_label": "cytoplasm",
  "term_id": "GO:0005737",
  "gene": "UniProtKB:Q92834"
}